{
  "term_id": "GO:0004383",
  "term_label": "guanylate cyclase activity",
  "gene": "UniProtKB:Q02108",
  "gene_name": "Guanylate cyclase soluble subunit alpha-1",
  "gene_symbol": "GUCY1A1"
}